host cell part [GO:0033643] (CC) Relationships: is a type of host cellular component [GO:0018995] Definition: Any constituent part of a host cell. The host is defined as the larger of the organisms involved in a symbiotic interaction. Note: Note that this term is in the subset of terms that should not be used for direct gene product annotation. Instead, select a child term or, if no appropriate child term exists, please request a new term. Direct annotations to this term may be amended during annotation QC. Subtypes: GO:0033644, GO:0033646, host cell postsynaptic membrane [GO:0035792], viral factory [GO:0039713], host intracellular region [GO:0043656], host peribacteroid membrane [GO:0043664], GO:0043665, host cell membrane pore complex [GO:0044084], host caveola [GO:0044155], host cell junction [GO:0044156], GO:0044157, host cell wall [GO:0044158], host cell synapse [GO:0044221], host cell surface [GO:0044228], host cell periplasmic space [GO:0044229], GO:0044230, host cell presynaptic membrane [GO:0044231], host cell periphery [GO:0044538], pathogen-containing vacuole [GO:0140220], GO:0140593 Sources: GOC:pamgo_curators